{
  "term_label": "DNA-binding transcription factor activity, RNA polymerase II-specific",
  "gene_name": "ATM interactor",
  "gene_symbol": "ATMIN",
  "term_id": "GO:0000981",
  "gene": "UniProtKB:O43313"
}